{
  "term_id": "UNKNOWN:0003",
  "gene_name": "Glutathione peroxidase 2",
  "gene": "UniProtKB:P18283",
  "gene_symbol": "GPX2",
  "term_label": "Unknown cellular component"
}